protein lysine deacetylase activity [GO:0033558] (molecular function) Also known as: protein deacetylase activity Relationships: is a type of deacetylase activity [GO:0019213]; is a type of catalytic activity, acting on a protein [GO:0140096] Definition: Catalysis of the reaction: Removal of an acetyl group from a lysine residue in a protein. References: PMID:27296530 Sources: RHEA:58108 Subtypes: histone deacetylase activity [GO:0004407], tubulin deacetylase activity [GO:0042903]